positive regulation of leukotriene production involved in inflammatory response [GO:0035491] (biological process) Sources: GOC:bf Definition: Any process that increases the rate, frequency or extent of the synthesis or release of any leukotriene following a stimulus as part of an inflammatory response. Relationships: is a type of regulation of leukotriene production involved in inflammatory response [GO:0035490]; is a type of GO:0050729; is_a GO:0051240; positively regulates leukotriene production involved in inflammatory response [GO:0002540]